regulation of lipoprotein metabolic process [GO:0050746] (biological process) Relationships: is a type of regulation of protein metabolic process [GO:0051246]; regulates lipoprotein metabolic process [GO:0042157] Sources: GOC:ai Subtypes: regulation of lipoprotein oxidation [GO:0034442], positive regulation of lipoprotein metabolic process [GO:0050747], negative regulation of lipoprotein metabolic process [GO:0050748], GO:1903059 Also known as: regulation of lipoprotein metabolism Definition: Any process that modulates the frequency, rate or extent of the chemical reactions and pathways involving lipoproteins, any conjugated, water-soluble protein in which the nonprotein group consists of a lipid or lipids.